{
  "gene_name": "Secretin",
  "term_label": "positive regulation of pancreatic juice secretion",
  "gene": "UniProtKB:P09683",
  "term_id": "GO:0090187",
  "gene_symbol": "SCT"
}